{
  "gene": "UniProtKB:Q99426",
  "term_label": "nucleus",
  "gene_symbol": "TBCB",
  "gene_name": "Tubulin-folding cofactor B",
  "term_id": "GO:0005634"
}